DNA-binding transcription factor binding [GO:0140297] (molecular function) Relationships: is a type of transcription factor binding [GO:0008134] Also known as: activating transcription factor binding, repressing transcription factor binding, transcription activator binding Definition: Binding to a DNA-binding transcription factor, a protein that interacts with a specific DNA sequence (sometimes referred to as a motif) within the regulatory region of a gene to modulate transcription. Sources: GOC:txnOH-2018 Subtypes: GO:0008140, bHLH transcription factor binding [GO:0043425], RNA polymerase II-specific DNA-binding transcription factor binding [GO:0061629]